{
  "term_id": "UNKNOWN:0001",
  "gene_name": "Nucleolar protein 10",
  "gene": "UniProtKB:Q9BSC4",
  "term_label": "Unknown molecular function",
  "gene_symbol": "NOL10"
}